{
  "term_id": "GO:0004713",
  "gene": "UniProtKB:P49761",
  "gene_symbol": "CLK3",
  "gene_name": "Dual specificity protein kinase CLK3",
  "term_label": "protein tyrosine kinase activity"
}